{
  "gene_symbol": "MARK1",
  "gene_name": "Serine_threonine-protein kinase MARK1",
  "gene": "UniProtKB:Q9P0L2",
  "term_label": "cytoplasm",
  "term_id": "GO:0005737"
}